{
  "gene": "UniProtKB:Q96DX8",
  "term_id": "GO:0005737",
  "term_label": "cytoplasm",
  "gene_name": "Receptor-transporting protein 4",
  "gene_symbol": "RTP4"
}